{
  "gene_symbol": "ZNF135",
  "gene_name": "Zinc finger protein 135",
  "gene": "UniProtKB:P52742",
  "term_id": "GO:0000981",
  "term_label": "DNA-binding transcription factor activity, RNA polymerase II-specific"
}